histone H2A methyltransferase activity [GO:0140940] (molecular function) Also known as: histone H2A methylase activity, histone H2A methylation Definition: Catalysis of the reaction: S-adenosyl-L-methionine + a histone H2 = S-adenosyl-L-homocysteine + a methylated histone H2A. Histone methylation generally occurs on either an arginine or a lysine residue. Relationships: is a type of histone methyltransferase activity [GO:0042054] Subtypes: histone H2AR3 methyltransferase activity [GO:0070612], histone H2AQ104 methyltransferase activity [GO:1990259] References: PMID:28450737